{
  "term_label": "Unknown cellular component",
  "gene_name": "Fibulin-1",
  "gene": "UniProtKB:P23142",
  "term_id": "UNKNOWN:0003",
  "gene_symbol": "FBLN1"
}